{
  "gene_symbol": "RWDD3",
  "gene_name": "RWD domain-containing protein 3",
  "term_label": "Unknown biological process",
  "gene": "UniProtKB:Q9Y3V2",
  "term_id": "UNKNOWN:0002"
}